{
  "term_id": "UNKNOWN:0001",
  "gene_name": "Protein NCBP2AS2",
  "gene_symbol": "NCBP2AS2",
  "gene": "UniProtKB:Q69YL0",
  "term_label": "Unknown molecular function"
}